{
  "term_id": "GO:0044458",
  "gene_symbol": "CFAP221",
  "term_label": "motile cilium assembly",
  "gene": "UniProtKB:Q4G0U5",
  "gene_name": "Cilia- and flagella-associated protein 221"
}